lipase binding [GO:0035473] (molecular function) Definition: Binding to a lipase. Sources: GOC:BHF Relationships: is a type of enzyme binding [GO:0019899]